natural killer cell activation involved in immune response [GO:0002323] (biological process) Also known as: NK cell activation during immune response, natural killer cell activation during immune response References: PMID:15032583 Sources: GOC:add Relationships: is a type of lymphocyte activation involved in immune response [GO:0002285]; is_a natural killer cell activation [GO:0030101]; BFO_0000050 innate immune response [GO:0045087] Definition: The change in morphology and behavior of a natural killer cell resulting from exposure a cytokine, chemokine, cellular ligand, or soluble factor, leading to the initiation or perpetuation of an immune response.